2-nitropropane catabolic process [GO:0046304] (biological process) Relationships: is_a xenobiotic catabolic process [GO:0042178] Sources: GOC:ai Definition: The chemical reactions and pathways resulting in the breakdown of 2-nitropropane, a clear, colorless liquid with a mild, fruity odor. Also known as: 2-nitropropane breakdown, 2-nitropropane catabolism, 2-nitropropane degradation